{
  "term_label": "G protein-coupled receptor activity",
  "gene": "UniProtKB:Q96P66",
  "gene_name": "Probable G-protein coupled receptor 101",
  "term_id": "GO:0004930",
  "gene_symbol": "GPR101"
}